{
  "term_label": "heterotrimeric G-protein complex",
  "term_id": "GO:0005834",
  "gene_symbol": "GNG3",
  "gene": "UniProtKB:P63215",
  "gene_name": "Guanine nucleotide-binding protein G(I)_G(S)_G(O) subunit gamma-3"
}